regulation of locomotor rhythm [GO:1904059] (biological process) Also known as: regulation of circadian locomotor activity rhythm Relationships: is a type of GO:0042752; is a type of regulation of behavior [GO:0050795]; RO_0002211 locomotor rhythm [GO:0045475] References: PMID:16310969 Sources: GOC:TermGenie, GO_REF:0000058 Definition: Any process that modulates the frequency, rate or extent of locomotor rhythm. Subtypes: GO:1904060, positive regulation of locomotor rhythm [GO:1904061]